positive regulation of long-chain fatty acid import into cell [GO:0140214] (biological process) Definition: Any process that activates or increases the frequency, rate or extent of long-chain fatty acid import into a cell. Subtypes: GO:0010747 References: PMID:28178239 Relationships: is a type of regulation of long-chain fatty acid import into cell [GO:0140212]; is a type of positive regulation of fatty acid transport [GO:2000193]; positively regulates long-chain fatty acid import into cell [GO:0044539]